{
  "gene_symbol": "KRT17",
  "term_label": "keratin filament",
  "gene_name": "Keratin, type I cytoskeletal 17",
  "gene": "UniProtKB:Q04695",
  "term_id": "GO:0045095"
}